{
  "term_label": "mitochondrion",
  "term_id": "GO:0005739",
  "gene_name": "Small ribosomal subunit protein uS10m",
  "gene_symbol": "MRPS10",
  "gene": "UniProtKB:P82664"
}